{
  "gene_symbol": "FLVCR1",
  "term_id": "GO:0006839",
  "gene": "UniProtKB:Q9Y5Y0",
  "term_label": "mitochondrial transport",
  "gene_name": "Heme transporter FLVCR1"
}